Edg-6 sphingosine 1-phosphate receptor binding [GO:0031759] (molecular function) Sources: GOC:mah, GOC:nln Also known as: Edg-6 sphingosine 1-phosphate receptor ligand Definition: Binding to an Edg-6 sphingosine 1-phosphate receptor. Relationships: is a type of endothelial differentiation G protein-coupled receptor binding [GO:0031753]